{
  "term_id": "UNKNOWN:0002",
  "gene_name": "Matrix-remodeling-associated protein 7",
  "term_label": "Unknown biological process",
  "gene_symbol": "MXRA7",
  "gene": "UniProtKB:P84157"
}